{
  "gene": "UniProtKB:Q9C0B6",
  "term_id": "GO:0021953",
  "gene_name": "BMP_retinoic acid-inducible neural-specific protein 2",
  "gene_symbol": "BRINP2",
  "term_label": "central nervous system neuron differentiation"
}